{
  "gene_name": "Poly(A) polymerase beta",
  "gene": "UniProtKB:Q9NRJ5",
  "term_label": "poly(A) RNA polymerase activity",
  "term_id": "GO:1990817",
  "gene_symbol": "PAPOLB"
}